{
  "term_label": "external side of plasma membrane",
  "term_id": "GO:0009897",
  "gene_symbol": "BTN3A3",
  "gene_name": "Butyrophilin subfamily 3 member A3",
  "gene": "UniProtKB:O00478"
}